{
  "gene_symbol": "BBS4",
  "term_label": "ciliary basal body",
  "term_id": "GO:0036064",
  "gene_name": "Bardet-Biedl syndrome 4 protein",
  "gene": "UniProtKB:Q96RK4"
}